transcriptional start site selection at RNA polymerase II promoter [GO:0001174] (biological process) Definition: Any process involved in the selection of the specific location within the template strand of an RNA polymerase II promoter for hybridization of the cognate ribonucleotides and formation of first phosphodiester bond within the nascent transcript. References: PMID:16826228, PMID:18846104 Sources: GOC:txnOH Relationships: is a type of DNA-templated transcriptional start site selection [GO:0001173]; is part of GO:0006367 Regulation: RO_0002211 by regulation of transcriptional start site selection at RNA polymerase II promoter [GO:0001178]